vesicle [GO:0031982] (cellular component) Definition: Any small, fluid-filled, spherical organelle enclosed by membrane. Sources: GOC:mah, GOC:pz, GOC:vesicles Also known as: membrane-bounded vesicle, membrane-enclosed vesicle Relationships: is a type of GO:0043227 Subtypes: GO:0097708, extracellular vesicle [GO:1903561]